{
  "gene_name": "Mitogen-activated protein kinase kinase kinase 14",
  "gene": "UniProtKB:Q99558",
  "term_label": "Unknown cellular component",
  "term_id": "UNKNOWN:0003",
  "gene_symbol": "MAP3K14"
}